{
  "gene": "UniProtKB:O00422",
  "gene_name": "Histone deacetylase complex subunit SAP18",
  "gene_symbol": "SAP18",
  "term_label": "transcription corepressor activity",
  "term_id": "GO:0003714"
}